striated muscle contraction involved in embryonic body morphogenesis [GO:0061199] (BP) Sources: GOC:dph, GOC:kmv Relationships: is a type of striated muscle contraction [GO:0006941]; is part of embryonic body morphogenesis [GO:0010172] Definition: The process in which force is generated within striated embryonic muscle tissue, resulting in a contraction of the muscle that contributes to the formation of an embryo's characteristic body morphology.